Aim21-Tda2 complex [GO:0110131] (cellular component) References: PMID:28706108, PMID:29467252 Sources: GOC:rn Definition: A complex that localizes to actin cortical patches at sites of endocytosis and negatively regulates barbed end F-actin assembly, resulting in the generation of free actin pools. The Aim21-Tda2 complex is necessary for efficient endocytosis and balancing the distribution of actin between patches and cables. Also known as: Aim21/Tda2 complex Relationships: is_a protein-containing complex [GO:0032991]; is part of actin cortical patch [GO:0030479]